{
  "gene_symbol": "TTTY12",
  "gene_name": "Putative transcript Y 12 protein",
  "term_id": "UNKNOWN:0001",
  "term_label": "Unknown molecular function",
  "gene": "UniProtKB:Q9BZ98"
}